{
  "gene_name": "Cyclin-dependent kinase 3",
  "term_id": "GO:0004693",
  "gene_symbol": "CDK3",
  "term_label": "cyclin-dependent protein serine/threonine kinase activity",
  "gene": "UniProtKB:Q00526"
}